{
  "gene_name": "BCL2_adenovirus E1B 19 kDa protein-interacting protein 3-like",
  "gene": "UniProtKB:O60238",
  "gene_symbol": "BNIP3L",
  "term_id": "GO:0005783",
  "term_label": "endoplasmic reticulum"
}